{
  "gene_symbol": "NEDD1",
  "gene": "UniProtKB:Q8NHV4",
  "gene_name": "Protein NEDD1",
  "term_id": "GO:0043015",
  "term_label": "gamma-tubulin binding"
}